positive regulation of synaptic transmission, glycinergic [GO:0060094] (biological process) Definition: Any process that activates or increases the frequency, rate or extent of glycinergic synaptic transmission. Glycinergic synaptic transmission is the process of communication from a neuron to another neuron across a synapse using the neurotransmitter glycine. Sources: GOC:dms, GOC:dph Also known as: positive regulation of glycinergic synaptic transmission Relationships: is a type of positive regulation of synaptic transmission [GO:0050806]; is a type of regulation of synaptic transmission, glycinergic [GO:0060092]; positively regulates synaptic transmission, glycinergic [GO:0060012] Subtypes: zinc potentiation of synaptic transmission, glycinergic [GO:0060095], positive regulation of glycine secretion, neurotransmission [GO:1904626]